{
  "gene": "UniProtKB:Q96RJ6",
  "gene_symbol": "FERD3L",
  "term_id": "GO:0000981",
  "gene_name": "Fer3-like protein",
  "term_label": "DNA-binding transcription factor activity, RNA polymerase II-specific"
}